{
  "gene": "UniProtKB:Q9NYP3",
  "gene_symbol": "DONSON",
  "term_label": "Unknown molecular function",
  "term_id": "UNKNOWN:0001",
  "gene_name": "Protein downstream neighbor of Son"
}